negative regulation of ductus arteriosus closure [GO:1904336] (biological process) Definition: Any process that stops, prevents or reduces the frequency, rate or extent of ductus arteriosus closure. Relationships: is a type of regulation of ductus arteriosus closure [GO:1904335]; is a type of negative regulation of artery morphogenesis [GO:1905652]; negatively regulates ductus arteriosus closure [GO:0097070] Also known as: down regulation of ductus arteriosus closure, down-regulation of ductus arteriosus closure, downregulation of ductus arteriosus closure, inhibition of ductus arteriosus closure References: PMID:16303610 Sources: GOC:TermGenie, GO_REF:0000058